{
  "gene_symbol": "ZNF850",
  "gene": "UniProtKB:A8MQ14",
  "gene_name": "Zinc finger protein 850",
  "term_label": "nucleus",
  "term_id": "GO:0005634"
}